{
  "term_id": "UNKNOWN:0001",
  "gene_name": "T cell receptor alpha variable 26-1",
  "gene": "UniProtKB:A0A087WT03",
  "term_label": "Unknown molecular function",
  "gene_symbol": "TRAV26-1"
}